{
  "gene": "UniProtKB:P49959",
  "term_label": "telomere maintenance",
  "term_id": "GO:0000723",
  "gene_symbol": "MRE11",
  "gene_name": "Double-strand break repair protein MRE11"
}